{
  "gene": "UniProtKB:Q5T653",
  "term_id": "GO:0032543",
  "gene_symbol": "MRPL2",
  "term_label": "mitochondrial translation",
  "gene_name": "Large ribosomal subunit protein uL2m"
}